{
  "term_id": "GO:0001755",
  "term_label": "neural crest cell migration",
  "gene_symbol": "SEMA4C",
  "gene_name": "Semaphorin-4C",
  "gene": "UniProtKB:Q9C0C4"
}